{
  "term_label": "Noc2p-Noc3p complex",
  "gene_symbol": "NOC2L",
  "term_id": "GO:0030691",
  "gene_name": "Nucleolar complex protein 2 homolog",
  "gene": "UniProtKB:Q9Y3T9"
}